{
  "term_id": "GO:0006357",
  "gene_symbol": "TOX4",
  "term_label": "regulation of transcription by RNA polymerase II",
  "gene": "UniProtKB:O94842",
  "gene_name": "TOX high mobility group box family member 4"
}